positive regulation of methane biosynthetic process from dimethylamine [GO:1900320] (biological process) Sources: GOC:TermGenie, GOC:mengo_curators Relationships: is a type of positive regulation of amine metabolic process [GO:0033240]; is a type of GO:1900318; is a type of positive regulation of alkane biosynthetic process [GO:1901579]; is_a positive regulation of cellular respiration [GO:1901857]; positively regulates methane biosynthetic process from dimethylamine [GO:2001129] Also known as: up regulation of methane biosynthetic process from dimethylamine, up-regulation of methane biosynthetic process from dimethylamine, upregulation of methane biosynthetic process from dimethylamine, activation of methane biosynthetic process from dimethylamine Definition: Any process that activates or increases the frequency, rate or extent of methane biosynthetic process from dimethylamine.